{
  "gene_symbol": "DENND1B",
  "term_id": "GO:0006897",
  "term_label": "endocytosis",
  "gene": "UniProtKB:Q6P3S1",
  "gene_name": "DENN domain-containing protein 1B"
}